{
  "term_id": "GO:0035329",
  "term_label": "hippo signaling",
  "gene_name": "MOB kinase activator 1B",
  "gene": "UniProtKB:Q7L9L4",
  "gene_symbol": "MOB1B"
}